threonine-phosphate decarboxylase activity [GO:0048472] (MF) Definition: Catalysis of the reaction: O-phospho-L-threonine + H+ = (R)-1-aminopropan-2-yl phosphate + CO2. Sources: EC:4.1.1.81, RHEA:11492 Also known as: L-threonine-O-3-phosphate decarboxylase activity, CobD, L-threonine O-3-phosphate carboxy-lyase [(R)-1-aminopropan-2-yl-phosphate-forming], L-threonine O-3-phosphate carboxy-lyase activity Relationships: is a type of carboxy-lyase activity [GO:0016831]